{
  "term_label": "DNA damage response",
  "gene_name": "Fanconi anemia core complex-associated protein 20",
  "term_id": "GO:0006974",
  "gene": "UniProtKB:Q6NZ36",
  "gene_symbol": "FAAP20"
}